{
  "gene_name": "cAMP-specific 3',5'-cyclic phosphodiesterase 4A",
  "term_label": "3',5'-cyclic-AMP phosphodiesterase activity",
  "gene_symbol": "PDE4A",
  "term_id": "GO:0004115",
  "gene": "UniProtKB:P27815"
}